{
  "gene_name": "Coiled-coil domain-containing protein 141",
  "gene": "UniProtKB:Q6ZP82",
  "term_id": "GO:0051963",
  "term_label": "regulation of synapse assembly",
  "gene_symbol": "CCDC141"
}